{
  "term_label": "ubiquitin protein ligase activity",
  "gene_name": "Probable E3 ubiquitin-protein ligase TRIML1",
  "gene": "UniProtKB:Q8N9V2",
  "gene_symbol": "TRIML1",
  "term_id": "GO:0061630"
}